{
  "gene": "UniProtKB:A0A5F9Z9Y6",
  "gene_symbol": "A0A5F9Z9Y6",
  "term_label": "transmembrane signaling receptor activity",
  "term_id": "GO:0004888",
  "gene_name": "Immunoglobulin subtype domain-containing protein"
}